{
  "term_label": "damaged DNA binding",
  "term_id": "GO:0003684",
  "gene_name": "Protein artemis",
  "gene": "UniProtKB:Q96SD1",
  "gene_symbol": "DCLRE1C"
}